{
  "gene_symbol": "MUC5AC",
  "term_id": "GO:0005615",
  "gene": "UniProtKB:P98088",
  "gene_name": "Mucin-5AC",
  "term_label": "extracellular space"
}